lipid A biosynthetic process [GO:0009245] (biological process) Definition: The chemical reactions and pathways resulting in the formation of lipid A, the glycolipid group of bacterial lipopolysaccharides, consisting of four to six fatty acyl chains linked to two glucosamine residues. Further modifications of the backbone are common. References: PMID:20974832, PMID:22216004 Sources: ISBN:0198506732 Also known as: lipid A anabolism, lipid A biosynthesis, lipid A formation, lipid A synthesis Relationships: is a type of phospholipid biosynthetic process [GO:0008654]; is a type of glycolipid biosynthetic process [GO:0009247]; is_a GO:0046493; is a type of lipooligosaccharide biosynthetic process [GO:1901271]